{
  "term_label": "Unknown biological process",
  "gene_symbol": "FAM240B",
  "gene_name": "Protein FAM240B",
  "gene": "UniProtKB:A0A1B0GVZ2",
  "term_id": "UNKNOWN:0002"
}